{
  "gene_name": "Putative UPF0633 protein LOC554249",
  "term_label": "Unknown molecular function",
  "term_id": "UNKNOWN:0001",
  "gene_symbol": "Q5XG85",
  "gene": "UniProtKB:Q5XG85"
}